{
  "gene": "UniProtKB:P54829",
  "term_id": "GO:0005886",
  "gene_name": "Tyrosine-protein phosphatase non-receptor type 5",
  "gene_symbol": "PTPN5",
  "term_label": "plasma membrane"
}